{
  "gene_symbol": "ATXN1L",
  "gene": "UniProtKB:P0C7T5",
  "term_label": "nucleus",
  "term_id": "GO:0005634",
  "gene_name": "Ataxin-1-like"
}